{
  "term_id": "GO:0035861",
  "gene": "UniProtKB:P35244",
  "gene_name": "Replication protein A 14 kDa subunit",
  "term_label": "site of double-strand break",
  "gene_symbol": "RPA3"
}